regulation of hair follicle maturation [GO:0048819] (biological process) Subtypes: negative regulation of hair follicle maturation [GO:0048817], positive regulation of hair follicle maturation [GO:0048818], regulation of timing of catagen [GO:0051794], regulation of timing of anagen [GO:0051884], GO:0051887 Sources: GOC:devbiol Relationships: is a type of regulation of developmental process [GO:0050793]; is a type of regulation of multicellular organismal process [GO:0051239]; regulates hair follicle maturation [GO:0048820] Definition: Any process that modulates the frequency, rate or extent of hair follicle maturation.